pyridoxamine transport [GO:0031922] (biological process) Definition: The directed movement of pyridoxamine into, out of or within a cell, or between cells, by means of some agent such as a transporter or pore. Pyridoxamine, 4-(aminomethyl)-5-(hydroxymethyl)-2-methylpyridin-3-ol, is one of the vitamin B6 compounds. Pyridoxal, pyridoxamine and pyridoxine are collectively known as vitamin B6, and are efficiently converted to the biologically active form of vitamin B6, pyridoxal phosphate. Sources: GOC:mah Relationships: is a type of organic cation transport [GO:0015695]; is a type of organic hydroxy compound transport [GO:0015850]; is a type of GO:0031919 Subtypes: GO:1903091